regulation of T-helper 17 cell differentiation [GO:2000319] (biological process) Sources: GOC:BHF, GOC:mah Relationships: is a type of regulation of T-helper cell differentiation [GO:0045622]; is a type of GO:2000316; regulates GO:0072539 Also known as: regulation of T-helper 17 cell development Subtypes: negative regulation of T-helper 17 cell differentiation [GO:2000320], positive regulation of T-helper 17 cell differentiation [GO:2000321], regulation of T-helper 17 cell lineage commitment [GO:2000328] Definition: Any process that modulates the frequency, rate or extent of T-helper 17 cell differentiation.